positive regulation of mitochondrial transcription [GO:1903109] (BP) References: PMID:21357609 Sources: GOC:TermGenie, GO_REF:0000058 Relationships: is a type of GO:0045893; is a type of regulation of mitochondrial transcription [GO:1903108]; positively regulates mitochondrial transcription [GO:0006390] Definition: Any process that activates or increases the frequency, rate or extent of transcription occurring in the mitochondrion. Also known as: positive regulation of transcription from mitochondrial promoter, up regulation of mitochondrial transcription, up regulation of transcription from mitochondrial promoter, up-regulation of mitochondrial transcription, up-regulation of transcription from mitochondrial promoter, upregulation of mitochondrial transcription, upregulation of transcription from mitochondrial promoter, activation of mitochondrial transcription, activation of transcription from mitochondrial promoter